{
  "term_label": "G protein-coupled adenosine receptor signaling pathway",
  "gene": "UniProtKB:P29274",
  "gene_name": "Adenosine receptor A2a",
  "gene_symbol": "ADORA2A",
  "term_id": "GO:0001973"
}